{
  "gene_name": "Isoleucine--tRNA ligase, cytoplasmic",
  "term_id": "GO:0004822",
  "term_label": "isoleucine-tRNA ligase activity",
  "gene_symbol": "IARS1",
  "gene": "UniProtKB:P41252"
}